{
  "gene_name": "Transmembrane epididymal protein 1",
  "term_id": "UNKNOWN:0001",
  "gene": "UniProtKB:Q5T9Z0",
  "gene_symbol": "TEDDM1",
  "term_label": "Unknown molecular function"
}